{
  "gene": "UniProtKB:Q9NVL8",
  "gene_name": "Uncharacterized protein CCDC198",
  "term_label": "Unknown cellular component",
  "gene_symbol": "CCDC198",
  "term_id": "UNKNOWN:0003"
}